{
  "gene": "UniProtKB:A0A1W2PPM0",
  "gene_symbol": "A0A1W2PPM0",
  "gene_name": "Uncharacterized protein",
  "term_id": "UNKNOWN:0001",
  "term_label": "Unknown molecular function"
}